{
  "gene_name": "Intraflagellar transport protein 80 homolog",
  "term_id": "UNKNOWN:0001",
  "term_label": "Unknown molecular function",
  "gene": "UniProtKB:Q9P2H3",
  "gene_symbol": "IFT80"
}